{
  "gene": "UniProtKB:Q9Y6R7",
  "term_id": "GO:0005201",
  "gene_symbol": "FCGBP",
  "gene_name": "IgGFc-binding protein",
  "term_label": "extracellular matrix structural constituent"
}